ribonucleoside triphosphate biosynthetic process [GO:0009201] (BP) Definition: The chemical reactions and pathways resulting in the formation of a ribonucleoside triphosphate, a compound consisting of a nucleobase linked to a ribose sugar esterified with triphosphate on the sugar. Sources: GOC:go_curators, ISBN:0198506732 Also known as: ribonucleoside triphosphate anabolism, ribonucleoside triphosphate biosynthesis, ribonucleoside triphosphate formation, ribonucleoside triphosphate synthesis Relationships: is a type of GO:0009142 Subtypes: purine ribonucleoside triphosphate biosynthetic process [GO:0009206], pyrimidine ribonucleoside triphosphate biosynthetic process [GO:0009209]